{
  "gene_name": "AT-rich interactive domain-containing protein 5A",
  "term_id": "GO:0005634",
  "gene": "UniProtKB:Q03989",
  "term_label": "nucleus",
  "gene_symbol": "ARID5A"
}